{
  "term_id": "GO:0005262",
  "gene": "UniProtKB:Q7Z443",
  "gene_symbol": "PKD1L3",
  "term_label": "calcium channel activity",
  "gene_name": "Polycystin-1-like protein 3"
}